antigen receptor-mediated signaling pathway [GO:0050851] (biological process) Definition: The series of molecular signals initiated by the cross-linking of an antigen receptor on a B or T cell. Sources: GOC:add Also known as: antigen receptor-mediated signalling pathway Relationships: is a type of immune response-activating cell surface receptor signaling pathway [GO:0002429] Subtypes: T cell receptor signaling pathway [GO:0050852], GO:0050853 Regulation: regulated by regulation of antigen receptor-mediated signaling pathway [GO:0050854]; positively regulated by positive regulation of antigen receptor-mediated signaling pathway [GO:0050857]; negatively regulated by GO:0050858